{
  "gene": "UniProtKB:Q15397",
  "term_label": "nucleolus",
  "term_id": "GO:0005730",
  "gene_name": "Pumilio homolog 3",
  "gene_symbol": "PUM3"
}